endoglycosylceramidase activity [GO:0047876] (molecular function) Definition: Catalysis of the reaction: H2O + oligoglycosylglucosylceramide = ceramide + oligoglycosylglucose. Also known as: EGCase activity, endo-glucosylceramidase activity, endoglycoceramidase activity, glycosyl-N-acetyl-sphingosine 1,1-beta-D-glucanohydrolase activity, oligoglycosylglucosylceramide glycohydrolase activity Relationships: is a type of GO:0004553 Sources: EC:3.2.1.123, MetaCyc:ENDOGLYCOSYLCERAMIDASE-RXN